{
  "term_label": "negative regulation of transcription by RNA polymerase II",
  "gene": "UniProtKB:Q9H0E3",
  "gene_name": "Histone deacetylase complex subunit SAP130",
  "term_id": "GO:0000122",
  "gene_symbol": "SAP130"
}